symbiont-mediated perturbation of host systemic acquired resistance [GO:0052160] (biological process) Definition: A process in which a symbiont alters or subverts systemic acquired resistance in the host organism; systemic acquired resistance is a salicylic acid-mediated response that confers broad spectrum systemic resistance. The host is defined as the larger of the organisms involved in a symbiotic interaction. Sources: GOC:mtg_pamgo_17jul06 Relationships: is a type of symbiont-mediated perturbation of host defense response [GO:0052031] Also known as: modulation by organism of systemic acquired resistance in other organism involved in symbiotic interaction, modulation by symbiont of host systemic acquired resistance, modulation by symbiont of systemic acquired resistance in host, perturbation of host systemic acquired resistance